transcription factor AP-1 complex [GO:0035976] (cellular component) Also known as: AP-1 complex, AP1 complex, Activating protein 1 complex, transcription factor AP1 complex Relationships: is a type of GO:0090575 Subtypes: GO:1990243 References: PMID:20060892, PMID:9069263 Sources: GOC:BHF, GOC:bf, GOC:rl, Wikipedia:AP-1_transcription_factor Definition: A heterodimeric transcription factor complex composed of proteins from the c-Fos, c-Jun, activating transcription factor (ATF) or JDP families. The subunits contain a basic leucine zipper (bZIP) domain that is essential for dimerization and DNA binding. Jun-Fos heterodimers bind preferentially to a heptamer consensus sequence (TPA responsive element (TRE)), whereas Jun-ATF dimers bind the cyclic AMP responsive element (CRE) to regulate transcription of target genes.